{
  "gene": "UniProtKB:O94921",
  "term_label": "nucleus",
  "gene_symbol": "CDK14",
  "term_id": "GO:0005634",
  "gene_name": "Cyclin-dependent kinase 14"
}